{
  "term_label": "nucleus",
  "gene": "UniProtKB:P63165",
  "gene_symbol": "SUMO1",
  "term_id": "GO:0005634",
  "gene_name": "Small ubiquitin-related modifier 1"
}